{
  "gene": "UniProtKB:Q8NCQ2",
  "gene_name": "Uncharacterized protein CSNK1G2-AS1",
  "term_id": "UNKNOWN:0001",
  "gene_symbol": "CSNK1G2-AS1",
  "term_label": "Unknown molecular function"
}